{
  "gene_symbol": "STK32A",
  "gene": "UniProtKB:Q8WU08",
  "term_id": "GO:0004674",
  "term_label": "protein serine/threonine kinase activity",
  "gene_name": "Serine_threonine-protein kinase 32A"
}